positive regulation of transcription by RNA polymerase I [GO:0045943] (biological process) Relationships: is a type of regulation of transcription by RNA polymerase I [GO:0006356]; is a type of positive regulation of DNA-templated transcription [GO:0045893]; positively regulates transcription by RNA polymerase I [GO:0006360] Subtypes: GO:1901838, positive regulation of termination of RNA polymerase I transcription [GO:2000732], positive regulation of transcription elongation by RNA polymerase I [GO:2001209] Also known as: positive regulation of transcription from Pol I promoter, positive regulation of transcription from RNA polymerase I promoter, up regulation of transcription from RNA polymerase I promoter, up-regulation of transcription from RNA polymerase I promoter, upregulation of transcription from RNA polymerase I promoter, activation of transcription from RNA polymerase I promoter, stimulation of transcription from RNA polymerase I promoter Definition: Any process that activates or increases the frequency, rate or extent of transcription mediated by RNA polymerase I. Sources: GOC:go_curators, GOC:txnOH